{
  "term_label": "transcription corepressor activity",
  "term_id": "GO:0003714",
  "gene_symbol": "SIN3B",
  "gene_name": "Paired amphipathic helix protein Sin3b",
  "gene": "UniProtKB:O75182"
}